{
  "term_id": "UNKNOWN:0001",
  "term_label": "Unknown molecular function",
  "gene_symbol": "Q6ZS92",
  "gene": "UniProtKB:Q6ZS92",
  "gene_name": "Putative uncharacterized protein FLJ45721"
}